proton-transporting V-type ATPase, V1 domain [GO:0033180] (cellular component) Relationships: is a type of GO:0033178; is part of proton-transporting V-type ATPase complex [GO:0033176] Subtypes: GO:0000221, plasma membrane proton-transporting V-type ATPase, V1 domain [GO:0000223] References: PMID:16449553 Sources: GOC:mah, ISBN:0716743663 Definition: A protein complex that forms part of a proton-transporting V-type ATPase and catalyzes ATP hydrolysis. The V1 complex consists of: (1) a globular headpiece with three alternating copies of subunits A and B that form a ring, (2) a central rotational stalk composed of single copies of subunits D and F, and (3) a peripheral stalk made of subunits C, E, G and H. Subunits A and B mediate the hydrolysis of ATP at three reaction sites associated with subunit A.